{
  "gene_name": "Golgi-associated RAB2 interactor protein 6",
  "term_label": "Unknown cellular component",
  "gene": "UniProtKB:Q8NEG0",
  "gene_symbol": "GARIN6",
  "term_id": "UNKNOWN:0003"
}